{
  "gene_symbol": "CSTPP1",
  "gene_name": "Centriolar satellite-associated tubulin polyglutamylase complex regulator 1",
  "gene": "UniProtKB:Q9H6J7",
  "term_id": "UNKNOWN:0002",
  "term_label": "Unknown biological process"
}